voltage-gated potassium channel activity involved in atrial cardiac muscle cell action potential repolarization [GO:0086089] (molecular function) Definition: Enables the transmembrane transfer of a potassium ion by a voltage-gated channel through the plasma membrane of an atrial cardiomyocyte contributing to the repolarization phase of an action potential. A voltage-gated channel is a channel whose open state is dependent on the voltage across the membrane in which it is embedded. Sources: GOC:BHF, GOC:mtg_cardiac_conduct_nov11 Also known as: voltage-gated potassium channel activity involved in atrial cardiomyocyte action potential repolarization Relationships: is_a GO:0086008; is part of atrial cardiac muscle cell action potential [GO:0086014]